{
  "gene": "UniProtKB:Q9BQT9",
  "term_id": "GO:0009986",
  "gene_name": "Calsyntenin-3",
  "term_label": "cell surface",
  "gene_symbol": "CLSTN3"
}